{
  "term_label": "RNA polymerase II cis-regulatory region sequence-specific DNA binding",
  "gene": "UniProtKB:O15060",
  "gene_name": "Zinc finger and BTB domain-containing protein 39",
  "gene_symbol": "ZBTB39",
  "term_id": "GO:0000978"
}